{
  "gene": "UniProtKB:Q8NEA4",
  "gene_name": "F-box only protein 36",
  "term_label": "Unknown molecular function",
  "gene_symbol": "FBXO36",
  "term_id": "UNKNOWN:0001"
}